{
  "term_label": "cytoplasm",
  "term_id": "GO:0005737",
  "gene_symbol": "PTPN22",
  "gene_name": "Tyrosine-protein phosphatase non-receptor type 22",
  "gene": "UniProtKB:Q9Y2R2"
}